methylphosphothioglycerate phosphatase activity [GO:0047382] (molecular function) Also known as: S-methyl-3-phospho-1-thio-D-glycerate phosphohydrolase activity, methylthiophosphoglycerate phosphatase activity Definition: Catalysis of the reaction: S-methyl-3-phospho-1-thio-D-glycerate + H2O = S-methyl-1-thio-D-glycerate + phosphate. Sources: EC:3.1.3.14, RHEA:16081 Relationships: is a type of GO:0016791